{
  "term_id": "GO:0004674",
  "term_label": "protein serine/threonine kinase activity",
  "gene_name": "Extracellular serine_threonine protein kinase FAM20C",
  "gene": "UniProtKB:Q8IXL6",
  "gene_symbol": "FAM20C"
}